{
  "gene": "UniProtKB:P41587",
  "term_label": "G protein-coupled peptide receptor activity",
  "term_id": "GO:0008528",
  "gene_symbol": "VIPR2",
  "gene_name": "Vasoactive intestinal polypeptide receptor 2"
}